pyridoxal metabolic process [GO:0042817] (biological process) Definition: The chemical reactions and pathways involving 3-hydroxy-5-(hydroxymethyl)-2-methyl-4-pyridinecarboxaldehyde, one of the vitamin B6 compounds. Pyridoxal, pyridoxamine and pyridoxine are collectively known as vitamin B6, and are efficiently converted to the biologically active form of vitamin B6, pyridoxal phosphate. References: PMID:21767669 Sources: GOC:jl Also known as: pyridoxal metabolism Subtypes: pyridoxal biosynthetic process [GO:0042821] Relationships: is a type of aldehyde metabolic process [GO:0006081]; is a type of vitamin B6 metabolic process [GO:0042816]